negative regulation of gamma-aminobutyric acid uptake involved in transmission of nerve impulse [GO:0051949] (biological process) Definition: Any process that stops, prevents, or reduces the frequency, rate or extent of the directed movement of gamma-aminobutyric acid (GABA, 4-aminobutyrate) into a neuron or glial cell. Also known as: down regulation of gamma-aminobutyric acid uptake during transmission of nerve impulse, down-regulation of gamma-aminobutyric acid uptake during transmission of nerve impulse, downregulation of gamma-aminobutyric acid uptake during transmission of nerve impulse, negative regulation of 4-aminobutyrate reuptake, negative regulation of 4-aminobutyrate uptake during transmission of nerve impulse, negative regulation of GABA reuptake, negative regulation of GABA uptake during transmission of nerve impulse, negative regulation of gamma-aminobutyric acid reuptake, negative regulation of gamma-aminobutyric acid uptake involved in conduction of nerve impulse, inhibition of gamma-aminobutyric acid uptake during transmission of nerve impulse, negative regulation of gamma-aminobutyric acid uptake during transmission of nerve impulse Sources: GOC:ai Relationships: is a type of GO:0032891; is a type of negative regulation of amino acid uptake involved in synaptic transmission [GO:0051942]; is_a regulation of gamma-aminobutyric acid uptake involved in transmission of nerve impulse [GO:0051947]; RO_0002212 gamma-aminobutyric acid reuptake [GO:0051936]